positive regulation of interleukin-9 production [GO:0032758] (biological process) Sources: GOC:mah Relationships: is a type of positive regulation of cytokine production [GO:0001819]; is a type of regulation of interleukin-9 production [GO:0032678]; positively regulates interleukin-9 production [GO:0032638] Definition: Any process that activates or increases the frequency, rate, or extent of interleukin-9 production. Also known as: positive regulation of IL-9 production, up regulation of interleukin-9 production, up-regulation of interleukin-9 production, upregulation of interleukin-9 production, activation of interleukin-9 production, positive regulation of interleukin-9 biosynthetic process, stimulation of interleukin-9 production